{
  "gene_symbol": "WNT9A",
  "term_id": "GO:0005125",
  "term_label": "cytokine activity",
  "gene_name": "Protein Wnt-9a",
  "gene": "UniProtKB:O14904"
}